{
  "gene_symbol": "SPOCK2",
  "gene_name": "Testican-2",
  "gene": "UniProtKB:Q92563",
  "term_label": "calcium ion binding",
  "term_id": "GO:0005509"
}